{
  "gene_name": "Mitogen-activated protein kinase 4",
  "term_label": "intracellular signal transduction",
  "gene_symbol": "MAPK4",
  "gene": "UniProtKB:P31152",
  "term_id": "GO:0035556"
}